sevenless binding [GO:0005118] (MF) Definition: Binding to a sevenless (sev) protein, a receptor tyrosine kinase. Relationships: is a type of signaling receptor binding [GO:0005102] Also known as: sev binding, sev ligand, sevenless ligand References: PMID:3151175 Sources: GOC:ceb